type 1 vasoactive intestinal polypeptide receptor binding [GO:0031891] (molecular function) Sources: GOC:mah, GOC:nln Definition: Binding to a type 1 vasoactive intestinal polypeptide receptor. Relationships: is a type of vasoactive intestinal polypeptide receptor binding [GO:0031890] Also known as: type 2 PACAP receptor binding, type 1 vasoactive intestinal polypeptide receptor ligand